{
  "gene_symbol": "TIMM10B",
  "gene": "UniProtKB:Q9Y5J6",
  "term_label": "protein insertion into mitochondrial inner membrane",
  "term_id": "GO:0045039",
  "gene_name": "Mitochondrial import inner membrane translocase subunit Tim10 B"
}